{
  "gene": "UniProtKB:Q96HV5",
  "term_id": "UNKNOWN:0001",
  "gene_symbol": "TMEM41A",
  "term_label": "Unknown molecular function",
  "gene_name": "Transmembrane protein 41A"
}